{
  "term_id": "GO:0045931",
  "gene": "UniProtKB:Q00987",
  "term_label": "positive regulation of mitotic cell cycle",
  "gene_name": "E3 ubiquitin-protein ligase Mdm2",
  "gene_symbol": "MDM2"
}